{
  "gene_name": "Immediate early response 3-interacting protein 1",
  "gene": "UniProtKB:Q9Y5U9",
  "term_id": "GO:0030134",
  "gene_symbol": "IER3IP1",
  "term_label": "COPII-coated ER to Golgi transport vesicle"
}